{
  "gene_name": "PR domain zinc finger protein 12",
  "gene": "UniProtKB:Q9H4Q4",
  "term_id": "GO:0010468",
  "term_label": "regulation of gene expression",
  "gene_symbol": "PRDM12"
}